{
  "term_label": "trans-Golgi network membrane",
  "gene_symbol": "TMEM79",
  "gene": "UniProtKB:Q9BSE2",
  "gene_name": "Transmembrane protein 79",
  "term_id": "GO:0032588"
}